negative regulation of octopamine signaling pathway [GO:2000129] (biological process) Definition: Any process that stops, prevents, or reduces the frequency, rate or extent of octopamine signaling pathway. Sources: GOC:mah Also known as: negative regulation of octopamine signalling pathway Relationships: is a type of negative regulation of octopamine or tyramine signaling pathway [GO:2000126]; is a type of regulation of octopamine signaling pathway [GO:2000128]; negatively regulates GO:0071927 Subtypes: negative regulation of octopamine signaling pathway involved in response to food [GO:2000140]